sn-2 acyl-lipid omega-3 desaturase (ferredoxin) activity [GO:0102993] (molecular function) Relationships: is a type of oxidoreductase activity, acting on paired donors, with oxidation of a pair of donors resulting in the reduction of molecular oxygen to two molecules of water [GO:0016717] Note: Introduces a cis double bond at a location 3 carbons away from the methyl end of the fatty acid. Acts on all 16:2- or 18:2-containing chloroplast membrane lipids, including phosphatidylglycerol, monogalactosyldiacylglycerol, digalactosyldiaclyglycerol, and sulfoquinovosyldiacylglycerol. Sources: EC:1.14.19.35 Definition: Catalysis of the reaction: a (9Z,12Z)-octadecadienoyl-containing glycerolipid + 2 H+ + O2 + 2 reduced [2Fe-2S]-[ferredoxin] = (9Z,12Z,15Z)-octadecatrienoyl-containing glycerolipid + 2 H2O + 2 oxidized [2Fe-2S]-[ferredoxin]. Also converts a (7Z,10Z)-hexadecadienoyl-containing glycerolipid into a (7Z,10Z,13Z)-hexadecatrienoyl-containing glycerolipid. Also known as: linolenate delta15 desaturase activity